{
  "term_label": "nucleus",
  "gene": "UniProtKB:O75688",
  "term_id": "GO:0005634",
  "gene_symbol": "PPM1B",
  "gene_name": "Protein phosphatase 1B"
}